{
  "gene": "UniProtKB:Q5SZQ8",
  "term_label": "mRNA binding",
  "term_id": "GO:0003729",
  "gene_symbol": "CELF3",
  "gene_name": "CUGBP Elav-like family member 3"
}